U1 snRNA binding [GO:0030619] (molecular function) Note: Note that this term may be useful for annotating other small nuclear RNAs (snRNAs). Definition: Binding to a U1 small nuclear RNA (U1 snRNA). Sources: GOC:mah Relationships: is a type of GO:0017069